{
  "term_label": "protein processing",
  "gene_name": "Neprilysin",
  "term_id": "GO:0016485",
  "gene": "UniProtKB:P08473",
  "gene_symbol": "MME"
}